5,6,7,8-tetrahydromethanopterin catabolic process [GO:1901284] (biological process) Sources: GOC:TermGenie, GOC:yaf, UniPathway:UPA00065 Definition: The chemical reactions and pathways resulting in the breakdown of 5,6,7,8-tetrahydromethanopterin. Relationships: is a type of GO:0006796; is a type of pteridine-containing compound catabolic process [GO:0042560]; is_a dicarboxylic acid catabolic process [GO:0043649]; is a type of organophosphate catabolic process [GO:0046434] Also known as: 5,6,7,8-tetrahydromethanopterin breakdown, 5,6,7,8-tetrahydromethanopterin catabolism, 5,6,7,8-tetrahydromethanopterin degradation